positive regulation of the force of heart contraction by neuronal epinephrine [GO:0003087] (BP) Sources: GOC:mtg_cardio Relationships: is a type of GO:0003059; is part of positive regulation of the force of heart contraction by neuronal epinephrine-norepinephrine [GO:0003090] Definition: The process in which the release of epinephrine from nerve endings modulates the force of heart muscle contraction. Also known as: increased force of heart contraction by epinephrine released from the nerve endings, increased force of heart contraction by neuronal epinephrine, increased force of heart contraction by neuronal adrenaline, positive regulation of heart contraction by adrenaline, positive regulation of heart contraction by neuronal epinephrine